{
  "gene_name": "Dihydrofolate reductase",
  "gene_symbol": "DHFR",
  "term_id": "GO:0005739",
  "gene": "UniProtKB:P00374",
  "term_label": "mitochondrion"
}